{
  "term_id": "GO:0006355",
  "term_label": "regulation of DNA-templated transcription",
  "gene_symbol": "PRMT2",
  "gene": "UniProtKB:P55345",
  "gene_name": "Protein arginine N-methyltransferase 2"
}